{
  "gene_name": "G protein-activated inward rectifier potassium channel 1",
  "term_label": "inward rectifier potassium channel activity",
  "gene_symbol": "KCNJ3",
  "term_id": "GO:0005242",
  "gene": "UniProtKB:P48549"
}